intramolecular aminotransferase activity [GO:0016869] (molecular function) Definition: Catalysis of the transfer of an amino group from one position to another within a single molecule. Also known as: intramolecular transferase activity, transferring amino groups Sources: GOC:mah Relationships: is a type of intramolecular transferase activity [GO:0016866] Subtypes: glutamate-1-semialdehyde 2,1-aminomutase activity [GO:0042286], D-lysine 5,6-aminomutase activity [GO:0047826], GO:0047831, L-leucine 2,3-aminomutase activity [GO:0050047], L-lysine 2,3-aminomutase activity [GO:0050066], L-tyrosine 2,3-aminomutase activity [GO:0050368]